flavanol binding [GO:0097245] (molecular function) Sources: GOC:sl Relationships: is_a flavonoid binding [GO:0097243]; is a type of GO:1901363 Subtypes: catechin binding [GO:0097246] Also known as: flavan-3-ol binding Definition: Binding to a flavanol.